{
  "gene_name": "Arylsulfatase J",
  "term_id": "UNKNOWN:0002",
  "term_label": "Unknown biological process",
  "gene_symbol": "ARSJ",
  "gene": "UniProtKB:Q5FYB0"
}